{
  "term_label": "actin cytoskeleton",
  "gene_symbol": "VIL1",
  "gene_name": "Villin-1",
  "gene": "UniProtKB:P09327",
  "term_id": "GO:0015629"
}